{
  "gene_symbol": "ITPR1",
  "gene_name": "Inositol 1,4,5-trisphosphate receptor type 1",
  "term_id": "GO:0005789",
  "term_label": "endoplasmic reticulum membrane",
  "gene": "UniProtKB:Q14643"
}